{
  "term_label": "fructose biosynthetic process",
  "gene_symbol": "SORD",
  "term_id": "GO:0046370",
  "gene_name": "Sorbitol dehydrogenase",
  "gene": "UniProtKB:Q00796"
}